negative regulation of midbrain dopaminergic neuron differentiation [GO:1904957] (biological process) Also known as: down regulation of DA neurogenesis from midbrain floor plate, down regulation of mDA neuron differentiation, down regulation of midbrain DA neurogenesis, down regulation of midbrain dopaminergic neuron differentiation, down regulation of midbrain dopaminergic neuron production, down-regulation of DA neurogenesis from midbrain floor plate, down-regulation of mDA neuron differentiation, down-regulation of midbrain DA neurogenesis, down-regulation of midbrain dopaminergic neuron differentiation, down-regulation of midbrain dopaminergic neuron production, downregulation of DA neurogenesis from midbrain floor plate, downregulation of mDA neuron differentiation, downregulation of midbrain DA neurogenesis, downregulation of midbrain dopaminergic neuron differentiation, downregulation of midbrain dopaminergic neuron production, negative regulation of DA neurogenesis from midbrain floor plate, negative regulation of mDA neuron differentiation, negative regulation of midbrain DA neurogenesis, negative regulation of midbrain dopaminergic neuron production, inhibition of DA neurogenesis from midbrain floor plate, inhibition of mDA neuron differentiation, inhibition of midbrain DA neurogenesis, inhibition of midbrain dopaminergic neuron differentiation, inhibition of midbrain dopaminergic neuron production Definition: Any process that stops, prevents or reduces the frequency, rate or extent of midbrain dopaminergic neuron differentiation. Sources: GOC:PARL, GOC:TermGenie, GOC:bf, GO_REF:0000058 Relationships: is a type of negative regulation of dopaminergic neuron differentiation [GO:1904339]; is a type of regulation of midbrain dopaminergic neuron differentiation [GO:1904956]; negatively regulates midbrain dopaminergic neuron differentiation [GO:1904948]